{
  "term_id": "GO:0008385",
  "term_label": "IkappaB kinase complex",
  "gene_symbol": "CHUK",
  "gene": "UniProtKB:O15111",
  "gene_name": "Inhibitor of nuclear factor kappa-B kinase subunit alpha"
}